{
  "gene": "UniProtKB:O95382",
  "term_id": "GO:0004709",
  "gene_symbol": "MAP3K6",
  "gene_name": "Mitogen-activated protein kinase kinase kinase 6",
  "term_label": "MAP kinase kinase kinase activity"
}